{
  "term_label": "Unknown molecular function",
  "gene": "UniProtKB:Q9UMZ3",
  "gene_name": "Phosphatidylinositol phosphatase PTPRQ",
  "gene_symbol": "PTPRQ",
  "term_id": "UNKNOWN:0001"
}